regulation of basement membrane organization [GO:0110011] (biological process) Definition: Any process that modulates the frequency, rate or extent of the assembly, disassembly or arrangement of constituent parts of the basement membrane. Relationships: is a type of regulation of extracellular matrix organization [GO:1903053]; regulates basement membrane organization [GO:0071711] Subtypes: GO:1904259 References: PMID:27404358 Sources: GOC:ha